{
  "gene_symbol": "SFTA2",
  "term_label": "Unknown molecular function",
  "gene_name": "Surfactant-associated protein 2",
  "gene": "UniProtKB:Q6UW10",
  "term_id": "UNKNOWN:0001"
}